exocrine system development [GO:0035272] (biological process) Definition: Progression of the exocrine system over time, from its formation to a mature structure. The exocrine system is a system of hormones and glands, where the glands secrete straight to a target site via ducts or tubes. The human exocrine system includes the salivary glands, sweat glands and many glands of the digestive system. Sources: GOC:bf, Wikipedia:Exocrine_gland Relationships: is_a system development [GO:0048731]